{
  "gene_name": "Solute carrier family 12 member 5",
  "gene": "UniProtKB:Q9H2X9",
  "gene_symbol": "SLC12A5",
  "term_label": "potassium:chloride symporter activity",
  "term_id": "GO:0015379"
}